regulation of cardiac endothelial to mesenchymal transition [GO:0061999] (biological process) Definition: Any process that modulates the frequency, rate or extent of cardiac endothelial to mesenchymal transition. Relationships: is a type of regulation of cell differentiation [GO:0045595]; regulates cardiac endothelial to mesenchymal transition [GO:0140074] References: PMID:26857067 Sources: GOC:BHF, GOC:BHF_miRNA, GOC:rph Subtypes: GO:0062000, GO:0062001